{
  "gene_symbol": "PLCB3",
  "term_label": "phosphatidylinositol-mediated signaling",
  "gene_name": "1-phosphatidylinositol 4,5-bisphosphate phosphodiesterase beta-3",
  "term_id": "GO:0048015",
  "gene": "UniProtKB:Q01970"
}